cyanidin 3-O-glucoside 2-O''-xylosyltransferase activity [GO:0102580] (molecular function) Relationships: is a type of GO:0016763 Sources: EC:2.4.2.51, GOC:pz Definition: Catalysis of the reaction: cyanidin 3-O-beta-D-glucoside betaine + UDP-alpha-D-xylose = cyanidin 3-O-beta-D-sambubioside + UDP.